{
  "gene": "UniProtKB:P20292",
  "gene_symbol": "ALOX5AP",
  "gene_name": "Arachidonate 5-lipoxygenase-activating protein",
  "term_id": "GO:0004602",
  "term_label": "glutathione peroxidase activity"
}